{
  "gene_symbol": "RTTN",
  "term_label": "ciliary basal body organization",
  "term_id": "GO:0032053",
  "gene": "UniProtKB:Q86VV8",
  "gene_name": "Rotatin"
}